neurotensin receptor binding [GO:0031846] (molecular function) Sources: GOC:mah, GOC:nln Relationships: is a type of neuropeptide receptor binding [GO:0071855] Also known as: neurotensin receptor ligand Subtypes: type 1 neurotensin receptor binding [GO:0031847] Definition: Binding to a neurotensin receptor.